{
  "gene_name": "DNA repair protein XRCC3",
  "term_label": "t-circle formation",
  "gene": "UniProtKB:O43542",
  "term_id": "GO:0090656",
  "gene_symbol": "XRCC3"
}